{
  "gene": "UniProtKB:Q6ZNB7",
  "gene_name": "Alkylglycerol monooxygenase",
  "gene_symbol": "AGMO",
  "term_id": "GO:0050479",
  "term_label": "glyceryl-ether monooxygenase activity"
}